{
  "gene_symbol": "PTPN9",
  "gene_name": "Tyrosine-protein phosphatase non-receptor type 9",
  "gene": "UniProtKB:P43378",
  "term_id": "UNKNOWN:0003",
  "term_label": "Unknown cellular component"
}